virion attachment to host cell pilus [GO:0039666] (biological process) Definition: The process by which a virion attaches to a host cell by binding to a pilus on the host cell surface. Pili are retractile filaments that protrude from gram-negative bacteria. Filamentous viruses can attach to the pilus tip, whereas icosahedral viruses can attach to the pilus side. Sources: UniProtKB-KW:KW-1175, VZ:981 Also known as: pilus-adsorption protein, pilus-mediated viral adsorption onto host cell, pilus-mediated viral attachment to host cell, viral attachment to host cell pilus Relationships: is a type of virion attachment to host cell [GO:0019062]; is part of GO:0046718